{
  "gene": "UniProtKB:Q9Y646",
  "term_label": "metallodipeptidase activity",
  "term_id": "GO:0070573",
  "gene_symbol": "CPQ",
  "gene_name": "Carboxypeptidase Q"
}